{
  "gene_name": "T-cell surface glycoprotein CD3 delta chain",
  "gene_symbol": "CD3D",
  "gene": "UniProtKB:P04234",
  "term_id": "GO:0045059",
  "term_label": "positive thymic T cell selection"
}